positive regulation of 1,2-propanediol catabolic process [GO:0160161] (biological process) Relationships: is a type of GO:1900421; positively regulates 1,2-propanediol catabolic process [GO:0051144] Definition: Any process that activates or increases the frequency, rate or extent of 1,2-propanediol catabolic process. Also known as: positive regulation of propanediol catabolic process References: PMID:7559322, PMID:9023178